{
  "gene_name": "E2F-associated phosphoprotein",
  "gene": "UniProtKB:Q56P03",
  "gene_symbol": "EAPP",
  "term_id": "GO:0005634",
  "term_label": "nucleus"
}